{
  "gene_name": "Sorting nexin-33",
  "term_label": "cleavage furrow formation",
  "term_id": "GO:0036089",
  "gene_symbol": "SNX33",
  "gene": "UniProtKB:Q8WV41"
}